mRNA capping enzyme complex [GO:0031533] (cellular component) Relationships: is a type of GO:0140513 Definition: A protein complex that consists of an RNA 5' triphosphatase and a guanyl transferase (Cet1p and Ceg1p in S. cerevisiae; Pct1 and Ceg1 in S. pombe) and is involved in mRNA capping. References: PMID:10347220, PMID:12455993, PMID:9345280 Sources: GOC:vw